{
  "gene_symbol": "OR52K1",
  "term_label": "olfactory receptor activity",
  "gene_name": "Olfactory receptor 52K1",
  "gene": "UniProtKB:Q8NGK4",
  "term_id": "GO:0004984"
}